{
  "gene_symbol": "ZFHX3",
  "term_label": "RNA polymerase II cis-regulatory region sequence-specific DNA binding",
  "gene_name": "Zinc finger homeobox protein 3",
  "term_id": "GO:0000978",
  "gene": "UniProtKB:Q15911"
}